{
  "term_label": "Unknown cellular component",
  "gene": "UniProtKB:Q96D53",
  "gene_symbol": "COQ8B",
  "term_id": "UNKNOWN:0003",
  "gene_name": "Atypical kinase COQ8B, mitochondrial"
}